midbrain-hindbrain boundary structural organization [GO:0021552] (biological process) Definition: The process that contributes to the act of creating the structural organization of the midbrain-hindbrain boundary structure. The midbrain-hindbrain domain of the embryonic brain is comprised of the mesencephalic vesicle and the first rhombencephalic vesicle at early somitogenesis stages. An organizing center at the boundary patterns the midbrain and hindbrain primordia of the neural plate. References: PMID:15541513 Sources: GOC:cls, GOC:dgh, GOC:dph, GOC:jid, GO_REF:0000021 Also known as: MHB structural organization, midbrain-hindbrain boundary structural organisation, isthmus structural organization Relationships: is a type of GO:0048532; is part of midbrain-hindbrain boundary morphogenesis [GO:0021555]